{
  "gene_symbol": "ATP6V1G2",
  "gene_name": "V-type proton ATPase subunit G 2",
  "term_id": "GO:0000221",
  "gene": "UniProtKB:O95670",
  "term_label": "vacuolar proton-transporting V-type ATPase, V1 domain"
}